{
  "term_id": "GO:0030667",
  "gene_name": "Islet cell autoantigen 1-like protein",
  "gene_symbol": "ICA1L",
  "term_label": "secretory granule membrane",
  "gene": "UniProtKB:Q8NDH6"
}